{
  "term_id": "GO:0005886",
  "gene_name": "Carcinoembryonic antigen-related cell adhesion molecule 6",
  "term_label": "plasma membrane",
  "gene": "UniProtKB:P40199",
  "gene_symbol": "CEACAM6"
}